{
  "gene_symbol": "ATP2B2",
  "term_label": "regulation of cytosolic calcium ion concentration",
  "gene_name": "Plasma membrane calcium-transporting ATPase 2",
  "gene": "UniProtKB:Q01814",
  "term_id": "GO:0051480"
}